{
  "gene": "UniProtKB:Q5TI25",
  "gene_name": "Neuroblastoma breakpoint family member 14",
  "term_id": "UNKNOWN:0003",
  "gene_symbol": "NBPF14",
  "term_label": "Unknown cellular component"
}